slit diaphragm [GO:0036057] (cellular component) References: PMID:12386277, PMID:15994232, PMID:18971929, PMID:19478094 Sources: GOC:mtg_kidney_jan10, GOC:rph Relationships: is a type of filtration diaphragm [GO:0036056] Definition: A specialized cell-cell junction found between the interdigitating foot processes of the glomerular epithelium (the podocytes) in the vertebrate kidney, which is adapted for facilitating glomerular filtration.